{
  "gene_name": "Rod cGMP-specific 3',5'-cyclic phosphodiesterase subunit alpha",
  "gene": "UniProtKB:P16499",
  "term_id": "GO:0042622",
  "term_label": "photoreceptor outer segment membrane",
  "gene_symbol": "PDE6A"
}